ornithine decarboxylase activity [GO:0004586] (molecular function) Definition: Catalysis of the reaction: L-ornithine + H+ = CO2 + putrescine. Sources: EC:4.1.1.17, RHEA:22964 Relationships: is_a carboxy-lyase activity [GO:0016831] Also known as: L-ornithine carboxy-lyase activity, L-ornithine carboxy-lyase (putrescine-forming), SpeC Regulation: negatively regulated by ornithine decarboxylase inhibitor activity [GO:0008073]; positively regulated by GO:0042978; regulated by ornithine decarboxylase regulator activity [GO:0042979]